{
  "gene_name": "Zinc finger protein 658",
  "term_label": "transcription cis-regulatory region binding",
  "term_id": "GO:0000976",
  "gene_symbol": "ZNF658",
  "gene": "UniProtKB:Q5TYW1"
}